{
  "gene": "UniProtKB:Q9HCJ1",
  "term_id": "UNKNOWN:0002",
  "term_label": "Unknown biological process",
  "gene_symbol": "ANKH",
  "gene_name": "Progressive ankylosis protein homolog"
}